prosaposin receptor activity [GO:0036505] (molecular function) Definition: Combining with prosaposin to initiate a change in cell activity. Prosaposin is the glycoprotein precursor of four cleavage products (saposins A, B, C and D). References: PMID:23690594, PMID:9388493 Sources: GOC:PARL, GOC:bf Relationships: is a type of G protein-coupled receptor activity [GO:0004930] Also known as: prosaposin-activated receptor activity